demethylmenaquinone methyltransferase activity [GO:0043770] (molecular function) References: PMID:1444716, PMID:9045837 Sources: RHEA:42640 Definition: Catalysis of the reaction: a 2-demethylmenaquinol + S-adenosyl-L-methionine = a menaquinol + H+ + S-adenosyl-L-homocysteine. Reaction substrates can have varying polyprenyl side chain length. Relationships: is a type of methyltransferase activity [GO:0008168]